{
  "term_id": "GO:0000981",
  "gene_name": "Zinc finger protein GLI2",
  "gene": "UniProtKB:P10070",
  "term_label": "DNA-binding transcription factor activity, RNA polymerase II-specific",
  "gene_symbol": "GLI2"
}